Ku-DNA ligase complex [GO:0070420] (cellular component) Relationships: is a type of GO:0070419 Definition: A nonhomologous end joining complex that contains one or more Ku monomers and one or more DNA ligase molecules from the LigC or LigD family, and mediates nonhomologous end joining in bacteria. References: PMID:17938628 Sources: GOC:mah